deep nuclear neuron cell migration [GO:0021946] (biological process) Definition: The directed movement of a deep nuclear neuron from the ventricular zone to the deep hindbrain nuclei. References: PMID:15157725 Sources: GOC:cls, GOC:dgh, GOC:dph, GOC:jid, GO_REF:0000021 Relationships: is a type of cell migration in hindbrain [GO:0021535]